{
  "term_label": "Golgi to plasma membrane protein transport",
  "gene_symbol": "ARFRP1",
  "term_id": "GO:0043001",
  "gene_name": "ADP-ribosylation factor-related protein 1",
  "gene": "UniProtKB:Q13795"
}